{
  "gene": "UniProtKB:A7E2F4",
  "term_label": "Golgi cisterna membrane",
  "term_id": "GO:0032580",
  "gene_symbol": "GOLGA8A",
  "gene_name": "Golgin subfamily A member 8A"
}